{
  "gene_name": "Mediator of RNA polymerase II transcription subunit 20",
  "gene_symbol": "MED20",
  "gene": "UniProtKB:Q9H944",
  "term_id": "GO:0016592",
  "term_label": "mediator complex"
}